{
  "gene_symbol": "SENP7",
  "term_label": "protein desumoylation",
  "gene_name": "Sentrin-specific protease 7",
  "term_id": "GO:0016926",
  "gene": "UniProtKB:Q9BQF6"
}